{
  "term_label": "Unknown molecular function",
  "gene_symbol": "EDF1",
  "gene": "UniProtKB:O60869",
  "term_id": "UNKNOWN:0001",
  "gene_name": "Endothelial differentiation-related factor 1"
}